{
  "gene_name": "Potassium voltage-gated channel subfamily KQT member 1",
  "term_label": "voltage-gated potassium channel activity involved in ventricular cardiac muscle cell action potential repolarization",
  "term_id": "GO:1902282",
  "gene": "UniProtKB:P51787",
  "gene_symbol": "KCNQ1"
}